{
  "term_id": "GO:0003823",
  "gene": "UniProtKB:A0A075B7E8",
  "gene_symbol": "IGHV3OR16-13",
  "gene_name": "Immunoglobulin heavy variable 3_OR16-13 (non-functional) (Fragment)",
  "term_label": "antigen binding"
}